{
  "term_id": "GO:0007259",
  "gene_symbol": "STAT5A",
  "gene": "UniProtKB:P42229",
  "term_label": "cell surface receptor signaling pathway via JAK-STAT",
  "gene_name": "Signal transducer and activator of transcription 5A"
}